host-mediated suppression of symbiont invasion [GO:0046597] (biological process) Also known as: blocking of symbiont entry into host cell, negative regulation of viral penetration into host cell, prevention of symbiont entry into host cell, negative regulation of viral entry into host cell, negative regulation of symbiont entry into host cell References: PMID:23544079 Definition: A process in which a host inhibits or disrupts the entry of a symbiont into a host cell. Relationships: is a type of innate immune response [GO:0045087]; is a type of host-mediated perturbation of symbiont process [GO:0051851]